{
  "gene_name": "Spermatogenesis-associated protein 6",
  "gene": "UniProtKB:Q9NWH7",
  "term_label": "myosin light chain binding",
  "gene_symbol": "SPATA6",
  "term_id": "GO:0032027"
}